{
  "term_id": "GO:0004996",
  "gene_name": "Thyrotropin receptor",
  "gene": "UniProtKB:P16473",
  "gene_symbol": "TSHR",
  "term_label": "thyroid-stimulating hormone receptor activity"
}